eukaryotic translation initiation factor 3 complex, eIF3m [GO:0071541] (cellular component) Definition: An eukaryotic translation initiation factor 3 complex that contains the PCI-domain protein eIF3m. References: PMID:15904532, PMID:19061185 Also known as: eIF3m-containing eukaryotic translation initiation factor 3 complex Relationships: is a type of eukaryotic translation initiation factor 3 complex [GO:0005852]